regulation of systemic arterial blood pressure by chemoreceptor signaling [GO:0001979] (BP) Also known as: chemoreceptor regulation of systemic arterial blood pressure, regulation of systemic arterial blood pressure by chemoreceptor signalling, chemoreceptor control of blood pressure Subtypes: regulation of systemic arterial blood pressure by carotid body chemoreceptor signaling [GO:0003027], regulation of systemic arterial blood pressure by aortic body chemoreceptor signaling [GO:0003028] Sources: GOC:dph, GOC:tb, ISBN:0721643949 Relationships: is_a nervous system process involved in regulation of systemic arterial blood pressure [GO:0001976] Definition: The process that modulates blood pressure by the action of chemoreceptors found in the carotid and aortic bodies and their resultant modulation of the vasomotor center. Chemoreceptors respond to oxygen, carbon dioxide and hydrogen ions.